{
  "gene_symbol": "FAM78B",
  "gene": "UniProtKB:Q5VT40",
  "term_label": "Unknown biological process",
  "gene_name": "Protein FAM78B",
  "term_id": "UNKNOWN:0002"
}